{
  "gene": "UniProtKB:P55289",
  "gene_symbol": "CDH12",
  "term_id": "GO:0007043",
  "term_label": "cell-cell junction assembly",
  "gene_name": "Cadherin-12"
}